small molecule metabolic process [GO:0044281] (BP) Subtypes: monosaccharide metabolic process [GO:0005996], alcohol metabolic process [GO:0006066], GO:0006082, GO:0006730, vitamin metabolic process [GO:0006766], dibenzofuran metabolic process [GO:0018893], dibenzo-p-dioxin metabolic process [GO:0018894], ammonia oxidation [GO:0019329], urea metabolic process [GO:0019627], small molecule catabolic process [GO:0044282], GO:0044283, formaldehyde metabolic process [GO:0046292], urate metabolic process [GO:0046415], dimethylsilanediol metabolic process [GO:0046454], GO:0055086, halogen metabolic process [GO:0070276], lactam metabolic process [GO:0072338], ketone body metabolic process [GO:1902224] Regulation: regulated by regulation of small molecule metabolic process [GO:0062012]; RO_0002213 by positive regulation of small molecule metabolic process [GO:0062013]; negatively regulated by negative regulation of small molecule metabolic process [GO:0062014] Note: Small molecules in GO include monosaccharides but exclude disaccharides and polysaccharides. Sources: GOC:curators, GOC:pde, GOC:vw Also known as: small molecule metabolism Definition: The chemical reactions and pathways involving small molecules, any low molecular weight, monomeric, non-encoded molecule. Relationships: is a type of metabolic process [GO:0008152]